{
  "gene_symbol": "ATXN2L",
  "term_id": "GO:0003729",
  "term_label": "mRNA binding",
  "gene_name": "Ataxin-2-like protein",
  "gene": "UniProtKB:Q8WWM7"
}